{
  "gene_name": "Putative uncharacterized protein URB1-AS1",
  "term_id": "UNKNOWN:0003",
  "gene": "UniProtKB:Q96HZ7",
  "term_label": "Unknown cellular component",
  "gene_symbol": "URB1-AS1"
}